{
  "gene_symbol": "NAB2",
  "gene": "UniProtKB:Q15742",
  "term_id": "GO:0003712",
  "gene_name": "NGFI-A-binding protein 2",
  "term_label": "transcription coregulator activity"
}